{
  "gene_symbol": "CAMK1G",
  "term_label": "signal transduction",
  "gene": "UniProtKB:Q96NX5",
  "term_id": "GO:0007165",
  "gene_name": "Calcium_calmodulin-dependent protein kinase type 1G"
}